phosphoglucokinase activity [GO:0050190] (molecular function) Also known as: ATP:D-glucose-1-phosphate 6-phosphotransferase activity, ATP:alpha-D-glucose-1-phosphate 6-phosphotransferase activity, glucose-phosphate kinase activity, phosphoglucokinase (phosphorylating) Sources: EC:2.7.1.10, RHEA:13377 Relationships: is a type of kinase activity [GO:0016301]; is a type of GO:0016773 Definition: Catalysis of the reaction: alpha-D-glucose 1-phosphate + ATP = alpha-D-glucose 1,6-bisphosphate + ADP + 2 H+.